{
  "gene": "UniProtKB:Q96H72",
  "term_id": "GO:0006882",
  "gene_name": "Zinc transporter ZIP13",
  "gene_symbol": "SLC39A13",
  "term_label": "intracellular zinc ion homeostasis"
}